{
  "gene_symbol": "IFNW1",
  "term_id": "GO:0005132",
  "gene": "UniProtKB:P05000",
  "term_label": "type I interferon receptor binding",
  "gene_name": "Interferon omega-1"
}